{
  "gene_name": "Calcium and integrin-binding family member 3",
  "term_label": "magnesium ion binding",
  "gene_symbol": "CIB3",
  "term_id": "GO:0000287",
  "gene": "UniProtKB:Q96Q77"
}